{
  "gene_symbol": "CSF3",
  "gene": "UniProtKB:P09919",
  "gene_name": "Granulocyte colony-stimulating factor",
  "term_label": "positive regulation of myeloid cell differentiation",
  "term_id": "GO:0045639"
}